{
  "gene": "UniProtKB:O43760",
  "gene_symbol": "SYNGR2",
  "gene_name": "Synaptogyrin-2",
  "term_id": "GO:0031594",
  "term_label": "neuromuscular junction"
}